{
  "gene": "UniProtKB:Q99572",
  "gene_symbol": "P2RX7",
  "term_label": "plasma membrane",
  "gene_name": "P2X purinoceptor 7",
  "term_id": "GO:0005886"
}